{
  "gene_name": "Cytoplasmic polyadenylation element-binding protein 2",
  "gene_symbol": "CPEB2",
  "term_id": "GO:0008135",
  "gene": "UniProtKB:Q7Z5Q1",
  "term_label": "translation factor activity, RNA binding"
}